striated muscle thin filament [GO:0005865] (cellular component) Relationships: is a type of myofilament [GO:0036379]; is part of actin cytoskeleton [GO:0015629]; is part of sarcomere [GO:0030017] Definition: Filaments formed of actin and associated proteins; attached to Z discs at either end of sarcomeres in myofibrils. Sources: ISBN:0815316194